{
  "term_label": "small GTPase-mediated signal transduction",
  "term_id": "GO:0007264",
  "gene_name": "Rho GTPase-activating protein 31",
  "gene": "UniProtKB:Q2M1Z3",
  "gene_symbol": "ARHGAP31"
}